pantetheine-phosphate adenylyltransferase activity [GO:0004595] (molecular function) Also known as: ATP:pantetheine-phosphate adenylyltransferase activity, phosphopantetheine adenylyltransferase activity, 3'-dephospho-CoA pyrophosphorylase activity, ATP:pantetheine-4'-phosphate adenylyltransferase activity, PPAT activity, dephospho-CoA diphosphorylase activity, dephospho-CoA pyrophosphorylase activity, dephospho-coenzyme A pyrophosphorylase activity, pantetheine phosphate adenylyltransferase activity Sources: EC:2.7.7.3, RHEA:19801 Definition: Catalysis of the reaction: ATP + pantetheine 4'-phosphate = 3'-dephospho-CoA + diphosphate. Relationships: is a type of adenylyltransferase activity [GO:0070566]